pseudouridine synthesis [GO:0001522] (BP) Definition: The intramolecular conversion of uridine to pseudouridine within an RNA molecule. Sources: GOC:hjd, GOC:mah Also known as: pseudouridylation Subtypes: rRNA pseudouridine synthesis [GO:0031118], tRNA pseudouridine synthesis [GO:0031119], snRNA pseudouridine synthesis [GO:0031120], mRNA pseudouridine synthesis [GO:1990481] Relationships: is a type of GO:0009451